{
  "gene": "UniProtKB:Q7RTP0",
  "gene_name": "Magnesium transporter NIPA1",
  "gene_symbol": "NIPA1",
  "term_id": "GO:0016020",
  "term_label": "membrane"
}